{
  "term_label": "anaphase-promoting complex",
  "gene": "UniProtKB:Q9BS18",
  "gene_symbol": "ANAPC13",
  "term_id": "GO:0005680",
  "gene_name": "Anaphase-promoting complex subunit 13"
}